{
  "gene_name": "Sodium-dependent organic anion transporter",
  "gene": "UniProtKB:Q3KNW5",
  "gene_symbol": "SLC10A6",
  "term_label": "Unknown cellular component",
  "term_id": "UNKNOWN:0003"
}